{
  "gene": "UniProtKB:Q71RH2",
  "gene_name": "Ceramide synthase",
  "term_label": "endoplasmic reticulum",
  "gene_symbol": "TLCD3B",
  "term_id": "GO:0005783"
}